{
  "gene_symbol": "AURKC",
  "gene_name": "Aurora kinase C",
  "gene": "UniProtKB:Q9UQB9",
  "term_id": "GO:0005634",
  "term_label": "nucleus"
}